{
  "term_id": "GO:0005762",
  "gene": "UniProtKB:Q9Y3B7",
  "gene_symbol": "MRPL11",
  "term_label": "mitochondrial large ribosomal subunit",
  "gene_name": "Large ribosomal subunit protein uL11m"
}